inner mitochondrial membrane protein complex [GO:0098800] (cellular component) Relationships: is a type of GO:0098796; is a type of mitochondrial protein-containing complex [GO:0098798]; is part of mitochondrial inner membrane [GO:0005743] Sources: GOC:dos Subtypes: PAM complex, Tim23 associated import motor [GO:0001405], TIM23 mitochondrial import inner membrane translocase complex [GO:0005744], m-AAA complex [GO:0005745], i-AAA complex [GO:0031942], GO:0032478, mitochondrial prohibitin complex [GO:0035632], mitochondrial inner membrane peptidase complex [GO:0042720], TIM22 mitochondrial import inner membrane insertion complex [GO:0042721], MICOS complex [GO:0061617], GO:0062011, MIB complex [GO:0140275], mitochondrial complex I intermediate assembly complex [GO:0160295], GO:1990246, INA complex [GO:1990524], GO:1990677, GO:7770001 Definition: Any protein complex that is part of the inner mitochondrial membrane.